outer dynein arm [GO:0036157] (CC) References: PMID:2557057, PMID:6218174 Sources: GOC:BHF, GOC:vk Relationships: is a type of GO:0005858 Definition: Outer arm structure present on the outer doublet microtubules of ciliary and flagellar axonemes. Outer dynein arms contain 2-3 heavy chains, two or more intermediate chains and a cluster of 4-8 light chains. Inner and outer dynein arms have different functions in the generation of microtubule-based motility. Also known as: outer dynein arm complex